regulation of ecdysteroid secretion [GO:0007555] (biological process) Definition: Any process that modulates the frequency, rate or extent of the regulated release of ecdysteroid from a cell. Sources: GOC:go_curators Relationships: is a type of regulation of steroid hormone secretion [GO:2000831]; regulates ecdysteroid secretion [GO:0045457] Subtypes: negative regulation of ecdysteroid secretion [GO:0045999], positive regulation of ecdysteroid secretion [GO:0046000]